{
  "gene_name": "Splicing regulator RBM11",
  "gene": "UniProtKB:P57052",
  "term_id": "GO:0003727",
  "gene_symbol": "RBM11",
  "term_label": "single-stranded RNA binding"
}